{
  "term_label": "extracellular matrix",
  "term_id": "GO:0031012",
  "gene": "UniProtKB:Q15389",
  "gene_name": "Angiopoietin-1",
  "gene_symbol": "ANGPT1"
}